cold-induced thermogenesis [GO:0106106] (biological process) Also known as: CIT Relationships: is_a temperature homeostasis [GO:0001659]; is a type of adaptive thermogenesis [GO:1990845] Definition: The process by which heat is generated by increasing metabolism in response to cold ambient temperatures in order to maintain a stable core body temperature. References: PMID:27876809 Regulation: RO_0002211 by regulation of cold-induced thermogenesis [GO:0120161]; positively regulated by positive regulation of cold-induced thermogenesis [GO:0120162]; negatively regulated by negative regulation of cold-induced thermogenesis [GO:0120163]